positive regulation of calcium-mediated signaling involved in cellular response to salt stress [GO:1901196] (biological process) Sources: GOC:TermGenie Also known as: positive regulation of calcium-mediated signaling involved in cellular response to ionic osmotic stress, positive regulation of calcium-mediated signaling involved in cellular salinity response, positive regulation of calcium-mediated signalling involved in cellular response to ionic osmotic stress, positive regulation of calcium-mediated signalling involved in cellular response to salt stress, positive regulation of calcium-mediated signalling involved in cellular salinity response, up regulation of calcium-mediated signaling involved in cellular response to ionic osmotic stress, up regulation of calcium-mediated signaling involved in cellular response to salt stress, up regulation of calcium-mediated signaling involved in cellular salinity response, up-regulation of calcium-mediated signaling involved in cellular response to ionic osmotic stress, up-regulation of calcium-mediated signaling involved in cellular response to salt stress, up-regulation of calcium-mediated signaling involved in cellular salinity response, upregulation of calcium-mediated signaling involved in cellular response to ionic osmotic stress, upregulation of calcium-mediated signaling involved in cellular response to salt stress, upregulation of calcium-mediated signaling involved in cellular salinity response, activation of calcium-mediated signaling involved in cellular response to ionic osmotic stress, activation of calcium-mediated signaling involved in cellular response to salt stress, activation of calcium-mediated signaling involved in cellular salinity response, stimulation of calcium-mediated signaling involved in cellular response to ionic osmotic stress, stimulation of calcium-mediated signaling involved in cellular response to salt stress, stimulation of calcium-mediated signaling involved in cellular salinity response Definition: Any positive regulation of calcium-mediated signaling that is involved in cellular response to salt stress. Relationships: is a type of positive regulation of calcium-mediated signaling [GO:0050850]; is part of cellular response to salt stress [GO:0071472]